sieve area [GO:0097217] (cellular component) Definition: A pit-like area in the cell wall of a sieve element; contains pores lined with callose and occupied by strands of protoplasmic material that interconnect the protoplasts of contiguous sieve elements. Note: Part of a sieve element (PO:0025406). Relationships: is a type of GO:0110165; BFO_0000050 plant-type cell wall [GO:0009505] Sources: ISBN:0471738433, POC:curators